{
  "gene_name": "Histone acetyltransferase KAT2A",
  "term_id": "GO:0140672",
  "gene_symbol": "KAT2A",
  "gene": "UniProtKB:Q92830",
  "term_label": "ATAC complex"
}